{
  "term_id": "GO:0005737",
  "term_label": "cytoplasm",
  "gene": "UniProtKB:Q15398",
  "gene_symbol": "DLGAP5",
  "gene_name": "Disks large-associated protein 5"
}